cytoskeleton-mediated cell swimming [GO:0071979] (biological process) References: PMID:18461074 Definition: Cell motility in which contractile cytoskeletal elements alter cell shape, resulting in the smooth movement of a cell through a liquid medium. Also known as: cytoskeleton-mediated swimming motility Relationships: is a type of cell swimming [GO:0071975]